{
  "term_id": "UNKNOWN:0001",
  "term_label": "Unknown molecular function",
  "gene": "UniProtKB:Q9Y2L5",
  "gene_symbol": "TRAPPC8",
  "gene_name": "Trafficking protein particle complex subunit 8"
}